{
  "term_id": "GO:0004864",
  "gene_name": "Proline-rich protein 3",
  "term_label": "protein phosphatase inhibitor activity",
  "gene": "UniProtKB:P79522",
  "gene_symbol": "PRR3"
}